{
  "term_label": "heteromeric SMAD protein complex",
  "gene_name": "Mothers against decapentaplegic homolog 2",
  "gene_symbol": "SMAD2",
  "gene": "UniProtKB:Q15796",
  "term_id": "GO:0071144"
}